{
  "term_label": "Unknown biological process",
  "term_id": "UNKNOWN:0002",
  "gene": "UniProtKB:Q9BSJ6",
  "gene_name": "Protein PIMREG",
  "gene_symbol": "PIMREG"
}